{
  "term_label": "establishment or maintenance of cell polarity",
  "gene_name": "Ras-related protein M-Ras",
  "gene_symbol": "MRAS",
  "gene": "UniProtKB:O14807",
  "term_id": "GO:0007163"
}